{
  "gene_symbol": "LILRB2",
  "term_label": "plasma membrane",
  "gene_name": "Leukocyte immunoglobulin-like receptor subfamily B member 2",
  "term_id": "GO:0005886",
  "gene": "UniProtKB:Q8N423"
}